vitamin D 23-hydroxylase activity [GO:0062179] (molecular function) Relationships: is a type of steroid hydroxylase activity [GO:0008395] Subtypes: 25-hydroxycholecalciferol-23-hydroxylase activity [GO:0062180], 1-alpha,25-dihydroxyvitamin D3 23-hydroxylase activity [GO:0062181] Definition: Catalysis of the hydroxylation of C-23 of any form of vitamin D. References: PMID:22100522, PMID:30205156